{
  "gene": "UniProtKB:Q92871",
  "term_id": "GO:0006013",
  "gene_name": "Phosphomannomutase 1",
  "term_label": "mannose metabolic process",
  "gene_symbol": "PMM1"
}